peptide-methionine (S)-S-oxide reductase activity [GO:0008113] (molecular function) Also known as: methionine sulfoxide (protein) reductase activity, peptide-methionine-(S)-S-oxide reductase activity, protein-methionine-S-oxide reductase activity Relationships: is a type of GO:0016671; is a type of catalytic activity, acting on a protein [GO:0140096] Definition: Catalysis of the reaction: L-methionyl-[protein] + [thioredoxin]-disulfide + H2O = L-methionyl-(S)-S-oxide-[protein] + [thioredoxin]-dithiol. Sources: RHEA:14217